{
  "gene_name": "Endophilin-A1",
  "gene_symbol": "SH3GL2",
  "term_id": "GO:0048488",
  "gene": "UniProtKB:Q99962",
  "term_label": "synaptic vesicle endocytosis"
}